positive regulation of CD8-positive, alpha-beta T cell proliferation [GO:2000566] (biological process) Definition: Any process that activates or increases the frequency, rate or extent of CD8-positive, alpha-beta T cell proliferation. Sources: GOC:obol Relationships: is a type of positive regulation of alpha-beta T cell proliferation [GO:0046641]; is a type of regulation of CD8-positive, alpha-beta T cell proliferation [GO:2000564]; is a type of positive regulation of CD8-positive, alpha-beta T cell activation [GO:2001187]; positively regulates CD8-positive, alpha-beta T cell proliferation [GO:0035740]